{
  "gene_symbol": "HSD17B11",
  "term_label": "steroid dehydrogenase activity",
  "term_id": "GO:0016229",
  "gene": "UniProtKB:Q8NBQ5",
  "gene_name": "Estradiol 17-beta-dehydrogenase 11"
}